{
  "gene_name": "E3 ubiquitin-protein ligase RNF220",
  "gene": "UniProtKB:Q5VTB9",
  "gene_symbol": "RNF220",
  "term_id": "GO:0061630",
  "term_label": "ubiquitin protein ligase activity"
}